{
  "term_id": "GO:0005886",
  "gene_symbol": "IL1R1",
  "gene": "UniProtKB:P14778",
  "gene_name": "Interleukin-1 receptor type 1",
  "term_label": "plasma membrane"
}